4-hydroxytryptamine kinase activity [GO:0140383] (molecular function) Relationships: is a type of kinase activity [GO:0016301] References: PMID:28763571 Definition: Catalysis of the reaction: 4-hydroxytryptamine + ATP = 4-hydoxytryptamine 4-phosphate + ADP + H+.